{
  "gene_name": "Chemerin-like receptor 2",
  "gene": "UniProtKB:P46091",
  "term_label": "plasma membrane",
  "term_id": "GO:0005886",
  "gene_symbol": "CMKLR2"
}